{
  "gene_symbol": "MARCKSL1",
  "term_id": "GO:0005737",
  "term_label": "cytoplasm",
  "gene": "UniProtKB:P49006",
  "gene_name": "MARCKS-related protein"
}